malate metabolic process [GO:0006108] (biological process) Also known as: malate metabolism Relationships: is_a dicarboxylic acid metabolic process [GO:0043648] Definition: The chemical reactions and pathways involving malate, the anion of hydroxybutanedioic acid, a chiral hydroxydicarboxylic acid. The (+) enantiomer is an important intermediate in metabolism as a component of both the TCA cycle and the glyoxylate cycle. Sources: ISBN:0198506732